positive regulation of photomorphogenesis [GO:2000306] (biological process) Definition: Any process that activates or increases the frequency, rate or extent of photomorphogenesis. Relationships: is a type of regulation of photomorphogenesis [GO:0010099]; is a type of GO:0048582; is a type of positive regulation of response to stimulus [GO:0048584]; positively regulates GO:0009640 Sources: GOC:obol Also known as: positive regulation of plant development in response to light